{
  "gene_name": "Solute carrier family 12 member 1",
  "term_id": "GO:0006884",
  "term_label": "cell volume homeostasis",
  "gene": "UniProtKB:Q13621",
  "gene_symbol": "SLC12A1"
}